regulation of synaptic transmission, glycinergic [GO:0060092] (biological process) Subtypes: GO:0060093, positive regulation of synaptic transmission, glycinergic [GO:0060094], regulation of glycine secretion, neurotransmission [GO:1904624] Relationships: is a type of modulation of chemical synaptic transmission [GO:0050804]; regulates synaptic transmission, glycinergic [GO:0060012] Definition: Any process that modulates the frequency, rate or extent of glycinergic synaptic transmission. Glycinergic synaptic transmission is the process of communication from a neuron to another neuron across a synapse using the neurotransmitter glycine. Sources: GOC:dms, GOC:dph